{
  "gene": "UniProtKB:Q8IWC1",
  "gene_name": "MAP7 domain-containing protein 3",
  "gene_symbol": "MAP7D3",
  "term_label": "microtubule cytoskeleton",
  "term_id": "GO:0015630"
}